{
  "gene": "UniProtKB:O94925",
  "gene_name": "Glutaminase kidney isoform, mitochondrial",
  "gene_symbol": "GLS",
  "term_label": "glutamate biosynthetic process",
  "term_id": "GO:0006537"
}